{
  "term_label": "Golgi apparatus",
  "gene": "UniProtKB:Q68CQ7",
  "gene_symbol": "GLT8D1",
  "gene_name": "Glycosyltransferase 8 domain-containing protein 1",
  "term_id": "GO:0005794"
}